{
  "gene": "UniProtKB:Q8NFQ8",
  "term_id": "GO:0061024",
  "gene_symbol": "TOR1AIP2",
  "term_label": "membrane organization",
  "gene_name": "Torsin-1A-interacting protein 2"
}